2,3-dihydroxybenzoate-serine ligase activity [GO:0047527] (molecular function) Relationships: is a type of acid-amino acid ligase activity [GO:0016881] Sources: EC:6.3.2.14 Definition: Catalysis of the reaction: ATP + 2,3-dihydroxybenzoate + L-serine = products of ATP breakdown + N-(2,3-dihydroxybenzoyl)-L-serine. Also known as: 2,3-dihydroxybenzoate:L-serine ligase activity, 2,3-dihydroxybenzoylserine synthetase activity, N-(2,3-dihydroxybenzoyl)-serine synthetase activity